iron ion transmembrane transporter activity [GO:0005381] (molecular function) Regulation: negatively regulated by GO:0097690 Subtypes: ferric iron transmembrane transporter activity [GO:0015091], ferrous iron transmembrane transporter activity [GO:0015093] Relationships: is a type of transition metal ion transmembrane transporter activity [GO:0046915]; is part of iron ion transmembrane transport [GO:0034755] Definition: Enables the transfer of iron (Fe) ions from one side of a membrane to the other. Note: An example of this is mouse ferroportin (UniProtKB:Q9JHI9), which transports iron out of the cell. Sources: GOC:ai Also known as: iron cation channel activity, iron channel activity, iron transporter activity, transmembrane iron ion permease activity, transmembrane iron permease activity, multicopper ferroxidase iron transport mediator activity, zinc, iron permease activity